{
  "term_id": "GO:0022627",
  "gene_name": "Putative ribosomal protein eS10-like",
  "term_label": "cytosolic small ribosomal subunit",
  "gene": "UniProtKB:Q9NQ39",
  "gene_symbol": "RPS10P5"
}